{
  "gene_symbol": "KCTD4",
  "gene": "UniProtKB:Q8WVF5",
  "term_label": "Unknown molecular function",
  "gene_name": "BTB_POZ domain-containing protein KCTD4",
  "term_id": "UNKNOWN:0001"
}